regulation of embryonic cell shape [GO:0016476] (biological process) Definition: Any process that modulates the surface configuration of an embryonic cell. Sources: GOC:dph, GOC:tb Also known as: shape changes of embryonic cells Relationships: is a type of GO:0008360; is a type of regulation of embryonic development [GO:0045995] Subtypes: dorsal closure, elongation of leading edge cells [GO:0007394]